pentose-phosphate shunt, non-oxidative branch [GO:0009052] (biological process) Also known as: pentose phosphate pathway, non-oxidative branch, pentose phosphate shunt, non-oxidative branch, pentose-phosphate pathway, non-oxidative branch Definition: The branch of the pentose-phosphate shunt which does not involve oxidation reactions. It comprises a series of sugar phosphate interconversions, starting with ribulose 5-P and producing fructose 6-P and glyceraldehyde 3-P. Sources: ISBN:0198506732, MetaCyc:NONOXIPENT-PWY Relationships: is_a generation of precursor metabolites and energy [GO:0006091]; is a type of glyceraldehyde-3-phosphate metabolic process [GO:0019682]; is part of pentose-phosphate shunt [GO:0006098]; has part D-ribulose-phosphate 3-epimerase activity [GO:0004750]; has part ribose-5-phosphate isomerase activity [GO:0004751]; has part transaldolase activity [GO:0004801]; has part transketolase activity [GO:0004802]